{
  "term_label": "maturation of LSU-rRNA from tricistronic rRNA transcript (SSU-rRNA, 5.8S rRNA, LSU-rRNA)",
  "gene_name": "Large ribosomal subunit protein uL30",
  "term_id": "GO:0000463",
  "gene_symbol": "RPL7",
  "gene": "UniProtKB:P18124"
}